{
  "term_label": "DNA-binding transcription repressor activity, RNA polymerase II-specific",
  "gene": "UniProtKB:Q6ZSB9",
  "gene_symbol": "ZBTB49",
  "term_id": "GO:0001227",
  "gene_name": "Zinc finger and BTB domain-containing protein 49"
}